metanephric ascending thin limb development [GO:0072218] (biological process) Definition: The process whose specific outcome is the progression of a metanephric ascending thin limb over time, from its formation to the mature structure. The metanephric ascending thin limb is a segment of a nephron tubule in the metanephros lying in the inner medulla that is permeable to ions but not to water and has a simple epithelium; active transepithelial solute transport is absent. Sources: GOC:mtg_kidney_jan10 Relationships: is a type of ascending thin limb development [GO:0072021]; is_a metanephric nephron tubule development [GO:0072234]; is part of metanephric loop of Henle development [GO:0072236]